{
  "gene_name": "E3 ubiquitin-protein ligase DTX4",
  "term_id": "GO:0016567",
  "gene": "UniProtKB:Q9Y2E6",
  "gene_symbol": "DTX4",
  "term_label": "protein ubiquitination"
}